{
  "term_label": "Unknown molecular function",
  "gene": "UniProtKB:Q5DID0",
  "gene_name": "Uromodulin-like 1",
  "term_id": "UNKNOWN:0001",
  "gene_symbol": "UMODL1"
}